{
  "gene": "UniProtKB:P52926",
  "gene_symbol": "HMGA2",
  "gene_name": "High mobility group protein HMGI-C",
  "term_label": "nucleus",
  "term_id": "GO:0005634"
}